{
  "gene_symbol": "IGFL4",
  "term_id": "UNKNOWN:0002",
  "term_label": "Unknown biological process",
  "gene": "UniProtKB:Q6B9Z1",
  "gene_name": "Insulin growth factor-like family member 4"
}